{
  "gene_symbol": "TRAJ52",
  "term_id": "UNKNOWN:0001",
  "gene_name": "T cell receptor alpha joining 52 (Fragment)",
  "term_label": "Unknown molecular function",
  "gene": "UniProtKB:A0A075B6W2"
}